{
  "term_label": "cytoplasm",
  "gene_name": "Aflatoxin B1 aldehyde reductase member 3",
  "gene_symbol": "AKR7A3",
  "term_id": "GO:0005737",
  "gene": "UniProtKB:O95154"
}